positive regulation of glial cell migration [GO:1903977] (BP) Subtypes: positive regulation of Schwann cell migration [GO:1900149], positive regulation of microglial cell migration [GO:1904141], positive regulation of astrocyte chemotaxis [GO:2000464] Also known as: positive regulation of glia cell migration, up regulation of glia cell migration, up regulation of glial cell migration, up-regulation of glia cell migration, up-regulation of glial cell migration, upregulation of glia cell migration, upregulation of glial cell migration, activation of glia cell migration, activation of glial cell migration Relationships: is a type of GO:0030335; is a type of regulation of glial cell migration [GO:1903975]; positively regulates glial cell migration [GO:0008347] Definition: Any process that activates or increases the frequency, rate or extent of glial cell migration. References: PMID:19100238 Sources: GOC:BHF, GOC:TermGenie, GOC:nc, GO_REF:0000058